glyoxylate reductase (NADH) activity [GO:0047964] (molecular function) Definition: Catalysis of the reaction: glycolate + NAD+ = glyoxylate + NADH. Relationships: is a type of GO:0106345 Sources: RHEA:18229 Also known as: NADH-dependent glyoxylate reductase activity, glycolate reductase activity, glyoxylic acid reductase activity